{
  "term_id": "GO:0036064",
  "gene_name": "Intraflagellar transport protein 140 homolog",
  "gene_symbol": "IFT140",
  "gene": "UniProtKB:Q96RY7",
  "term_label": "ciliary basal body"
}